{
  "gene_symbol": "PLPP2",
  "gene": "UniProtKB:O43688",
  "gene_name": "Phospholipid phosphatase 2",
  "term_id": "GO:0007165",
  "term_label": "signal transduction"
}